MAP kinase kinase kinase activity [GO:0004709] (molecular function) Relationships: is a type of GO:0004674; is part of MAPK cascade [GO:0000165] References: PMID:9561267 Definition: Catalysis of the phosphorylation and activation of a MAP kinase kinase; each MAP kinase kinase can be phosphorylated by any of several MAP kinase kinase kinases. Also known as: MAPK/ERK kinase kinase activity, MEKK activity, MLK-like mitogen-activated protein triple kinase activity, ATP:protein phosphotransferase (MAPKKKK-activated) activity, MAP3K, MAPKKK activity, MEK kinase activity, MEKK, MEKK1, MEKK2, MEKK3, MLTK, MLTKa, MLTKb, Mil/Raf, REKS, STK28, cMos, cRaf, mitogen-activated protein kinase kinase kinase activity Subtypes: GO:0004706